{
  "term_label": "cell surface receptor signaling pathway",
  "term_id": "GO:0007166",
  "gene_symbol": "TNFSF14",
  "gene_name": "Tumor necrosis factor ligand superfamily member 14",
  "gene": "UniProtKB:O43557"
}